1,2-dihydrovomilenine reductase activity [GO:0050615] (molecular function) Definition: Catalysis of the reaction: 17-O-acetylnorajmaline + NADP+ = 1,2-dihydrovomilenine + H+ + NADPH. Also known as: 17-O-acetylnorajmaline:NADP+ oxidoreductase activity Relationships: is a type of oxidoreductase activity, acting on the CH-CH group of donors, NAD or NADP as acceptor [GO:0016628] Sources: EC:1.3.1.73, RHEA:12320